{
  "gene_symbol": "GAK",
  "gene": "UniProtKB:O14976",
  "term_id": "GO:0072318",
  "term_label": "clathrin coat disassembly",
  "gene_name": "Cyclin-G-associated kinase"
}